{
  "gene": "UniProtKB:P01876",
  "term_id": "GO:0006958",
  "term_label": "complement activation, classical pathway",
  "gene_name": "Immunoglobulin heavy constant alpha 1",
  "gene_symbol": "IGHA1"
}